{
  "term_id": "UNKNOWN:0001",
  "gene": "UniProtKB:Q01954",
  "gene_symbol": "BNC1",
  "term_label": "Unknown molecular function",
  "gene_name": "Zinc finger protein basonuclin-1"
}